{
  "term_id": "GO:0000981",
  "gene_symbol": "ZBTB7A",
  "gene_name": "Zinc finger and BTB domain-containing protein 7A",
  "gene": "UniProtKB:O95365",
  "term_label": "DNA-binding transcription factor activity, RNA polymerase II-specific"
}